{
  "term_id": "GO:0071037",
  "gene_name": "Zinc finger CCHC domain-containing protein 7",
  "gene": "UniProtKB:Q8N3Z6",
  "term_label": "nuclear polyadenylation-dependent snRNA catabolic process",
  "gene_symbol": "ZCCHC7"
}